regulation of cell projection size [GO:0032536] (biological process) Definition: A process that modulates the size of a cell projection. Sources: GOC:mah Relationships: is a type of GO:0032535 Subtypes: regulation of axon diameter [GO:0031133], regulation of microvillus length [GO:0032532]